peroxisome transport along microtubule [GO:0036250] (biological process) References: PMID:21525035 Sources: GOC:pm Relationships: is a type of organelle transport along microtubule [GO:0072384] Definition: The directed movement of a peroxisome along a microtubule, mediated by motor proteins.